{
  "term_id": "UNKNOWN:0001",
  "term_label": "Unknown molecular function",
  "gene": "UniProtKB:A0A0A0MT86",
  "gene_symbol": "IGLJ5",
  "gene_name": "Immunoglobulin lambda joining 5 (non-functional) (Fragment)"
}